membrane scission GTPase motor activity [GO:1990606] (molecular function) Definition: Generation of a 'twisting' activity resulting in the scission of a membrane, driven by GTP hydrolysis. Relationships: is a type of GTPase motor activity [GO:0061791] References: PMID:11242086, PMID:23530241, PMID:24515348